very long-chain fatty-acyl-CoA catabolic process [GO:0036113] (biological process) Also known as: very long-chain fatty-acyl-CoA breakdown, very long-chain fatty-acyl-CoA catabolism, very long-chain fatty-acyl-CoA degradation Relationships: is_a very long-chain fatty-acyl-CoA metabolic process [GO:0036111]; is a type of fatty-acyl-CoA catabolic process [GO:0036115] Note: While there is not universal consensus on the lengths of short-, medium-, long- and very-long-chain fatty acids, the GO uses the definitions in ChEBI (see CHEBI:26666, CHEBI:59554, CHEBI:15904 and CHEBI:27283). Definition: The chemical reactions and pathways resulting in the breakdown of very long-chain fatty-acyl-CoAs, any derivative of coenzyme A in which the sulfhydryl group is in a thioester linkage with a very long-chain fatty-acyl group. A very long-chain fatty acid has an aliphatic tail containing more than 22 carbons. Sources: GOC:pm